phialide development [GO:0070790] (biological process) References: PMID:9529886 Relationships: is a type of GO:0003006; is a type of GO:0048468; is part of GO:0070787 Also known as: development of secondary sterigmata Definition: The process whose specific outcome is the progression of phialides over time, from its formation to the mature structure. Phialides are specialized cells that bud from the ends of metulae on the conidiophore tip. Chains of conidia, or asexual spores, develop from the phialide tips. Regulation: regulated by regulation of phialide development [GO:0070805]; RO_0002212 by negative regulation of phialide development [GO:0070806]; positively regulated by positive regulation of phialide development [GO:0070807]